{
  "gene_symbol": "TRAJ53",
  "term_label": "Unknown biological process",
  "gene_name": "T cell receptor alpha joining 53 (Fragment)",
  "term_id": "UNKNOWN:0002",
  "gene": "UniProtKB:A0A075B6W9"
}